{
  "gene_name": "Putative protein BCE-1",
  "term_id": "UNKNOWN:0003",
  "gene": "UniProtKB:O60756",
  "gene_symbol": "BCE1",
  "term_label": "Unknown cellular component"
}